{
  "term_id": "GO:0005739",
  "gene_name": "Cobalamin trafficking protein CblD",
  "term_label": "mitochondrion",
  "gene_symbol": "MMADHC",
  "gene": "UniProtKB:Q9H3L0"
}